{
  "term_id": "GO:0042262",
  "gene_symbol": "NUDT1",
  "gene": "UniProtKB:P36639",
  "term_label": "DNA protection",
  "gene_name": "Oxidized purine nucleoside triphosphate hydrolase"
}